{
  "term_id": "GO:0006357",
  "gene_symbol": "MED17",
  "gene_name": "Mediator of RNA polymerase II transcription subunit 17",
  "gene": "UniProtKB:Q9NVC6",
  "term_label": "regulation of transcription by RNA polymerase II"
}